{
  "gene": "UniProtKB:Q9P0S3",
  "gene_name": "ORM1-like protein 1",
  "gene_symbol": "ORMDL1",
  "term_label": "sphingolipid biosynthetic process",
  "term_id": "GO:0030148"
}